{
  "gene_symbol": "PPP2R2D",
  "term_id": "GO:0000159",
  "gene": "UniProtKB:Q66LE6",
  "gene_name": "Serine_threonine-protein phosphatase 2A 55 kDa regulatory subunit B delta isoform",
  "term_label": "protein phosphatase type 2A complex"
}